NADH kinase activity [GO:0042736] (molecular function) Definition: Catalysis of the reaction: ATP + NADH = ADP + 2 H+ + NADPH. Sources: EC:2.7.1.86, RHEA:12260 Also known as: ATP:NADH 2'-phosphotransferase activity, DPNH kinase activity, reduced diphosphopyridine nucleotide kinase activity, reduced nicotinamide adenine dinucleotide kinase (phosphorylating) Relationships: is a type of kinase activity [GO:0016301]; is a type of phosphotransferase activity, alcohol group as acceptor [GO:0016773]